{
  "term_label": "nucleus",
  "gene_name": "Atrophin-1",
  "gene": "UniProtKB:P54259",
  "gene_symbol": "ATN1",
  "term_id": "GO:0005634"
}